{
  "term_label": "Unknown molecular function",
  "gene": "UniProtKB:Q13772",
  "gene_name": "Nuclear receptor coactivator 4",
  "gene_symbol": "NCOA4",
  "term_id": "UNKNOWN:0001"
}